{
  "term_id": "GO:0005615",
  "gene": "UniProtKB:Q15726",
  "gene_symbol": "KISS1",
  "gene_name": "Metastasis-suppressor KiSS-1",
  "term_label": "extracellular space"
}